{
  "gene": "UniProtKB:P04183",
  "gene_symbol": "TK1",
  "gene_name": "Thymidine kinase, cytosolic",
  "term_id": "UNKNOWN:0003",
  "term_label": "Unknown cellular component"
}